{
  "gene_symbol": "CCDC192",
  "gene": "UniProtKB:P0DO97",
  "gene_name": "Coiled-coil domain-containing protein 192",
  "term_label": "Unknown molecular function",
  "term_id": "UNKNOWN:0001"
}